{
  "term_label": "collagen type I trimer",
  "gene_symbol": "COL1A2",
  "gene": "UniProtKB:P08123",
  "term_id": "GO:0005584",
  "gene_name": "Collagen alpha-2(I) chain"
}